{
  "term_id": "GO:0005737",
  "term_label": "cytoplasm",
  "gene": "UniProtKB:Q969S8",
  "gene_name": "Polyamine deacetylase HDAC10",
  "gene_symbol": "HDAC10"
}